{
  "term_id": "GO:0007264",
  "gene": "UniProtKB:Q8IWW6",
  "term_label": "small GTPase-mediated signal transduction",
  "gene_name": "Rho GTPase-activating protein 12",
  "gene_symbol": "ARHGAP12"
}